response to triterpenoid [GO:1905836] (biological process) Relationships: is a type of GO:0033993 References: PMID:28078994 Sources: GOC:TermGenie, GO_REF:0000071 Definition: Any process that results in a change in state or activity of a cell or an organism (in terms of movement, secretion, enzyme production, gene expression, etc.) as a result of a triterpenoid stimulus. Subtypes: GO:1905092, cellular response to triterpenoid [GO:1905837]